sulfite reductase (NADPH) activity [GO:0004783] (MF) Sources: RHEA:13801 Also known as: sulphite reductase (NADPH) activity, H2S-NADP oxidoreductase activity, NADPH-dependent sulfite reductase activity, NADPH-sulfite reductase activity, NADPH:sulfite reductase flavoprotein, hydrogen-sulfide:NADP+ oxidoreductase activity, sulfite (reduced nicotinamide adenine dinucleotide phosphate) reductase activity Relationships: is_a sulfite reductase activity [GO:0016002]; is a type of oxidoreductase activity, acting on a sulfur group of donors, NAD(P) as acceptor [GO:0016668] Definition: Catalysis of the reaction: hydrogen sulfide + 3 NADP+ + 3 H2O = sulfite + 3 NADPH + 3 H+.